{
  "term_id": "UNKNOWN:0003",
  "gene_symbol": "CT55",
  "gene": "UniProtKB:Q8WUE5",
  "gene_name": "Cancer_testis antigen 55",
  "term_label": "Unknown cellular component"
}